{
  "term_label": "Unknown cellular component",
  "gene": "UniProtKB:Q32M92",
  "gene_symbol": "C15orf32",
  "term_id": "UNKNOWN:0003",
  "gene_name": "Uncharacterized protein C15orf32"
}